{
  "gene_name": "Homeobox protein Hox-D11",
  "term_label": "regulation of transcription by RNA polymerase II",
  "gene_symbol": "HOXD11",
  "term_id": "GO:0006357",
  "gene": "UniProtKB:P31277"
}